{
  "term_label": "maintenance of gastrointestinal epithelium",
  "term_id": "GO:0030277",
  "gene_symbol": "CRACD",
  "gene_name": "Capping protein-inhibiting regulator of actin dynamics",
  "gene": "UniProtKB:Q6ZU35"
}